{
  "gene_symbol": "NME7",
  "term_id": "GO:0005879",
  "gene": "UniProtKB:Q9Y5B8",
  "term_label": "axonemal microtubule",
  "gene_name": "Nucleoside diphosphate kinase 7"
}